{
  "term_label": "heart development",
  "gene_name": "Lysine-specific demethylase 6B",
  "gene_symbol": "KDM6B",
  "term_id": "GO:0007507",
  "gene": "UniProtKB:O15054"
}